{
  "gene": "UniProtKB:Q96RQ1",
  "gene_symbol": "ERGIC2",
  "gene_name": "Endoplasmic reticulum-Golgi intermediate compartment protein 2",
  "term_id": "GO:0016020",
  "term_label": "membrane"
}